maturation of LSU-rRNA from tetracistronic rRNA transcript (SSU-rRNA, LSU-rRNA, 4.5S-rRNA, 5S-rRNA) [GO:0000488] (biological process) Sources: GOC:curators Definition: Any process involved in the maturation of a precursor Large SubUnit (LSU) ribosomal RNA (rRNA) molecule into a mature LSU-rRNA molecule from the pre-rRNA molecule originally produced as a tetracistronic rRNA transcript that contains the Small Subunit (SSU) rRNA, Large Subunit (LSU) the 4.5S rRNA, and the 5S rRNA in that order from 5' to 3' along the primary transcript. Relationships: is a type of maturation of LSU-rRNA [GO:0000470]